{
  "gene_name": "Large ribosomal subunit protein uL15m",
  "term_id": "GO:0003735",
  "gene": "UniProtKB:Q9P015",
  "term_label": "structural constituent of ribosome",
  "gene_symbol": "MRPL15"
}